{
  "gene_name": "Transcription elongation factor A protein-like 9",
  "gene_symbol": "TCEAL9",
  "term_id": "UNKNOWN:0002",
  "term_label": "Unknown biological process",
  "gene": "UniProtKB:Q9UHQ7"
}